regulation of mitochondrial electron transport, NADH to ubiquinone [GO:1902956] (BP) Subtypes: negative regulation of mitochondrial electron transport, NADH to ubiquinone [GO:1902957], positive regulation of mitochondrial electron transport, NADH to ubiquinone [GO:1902958] Relationships: is a type of regulation of aerobic respiration [GO:1903715]; regulates mitochondrial electron transport, NADH to ubiquinone [GO:0006120] Definition: Any process that modulates the frequency, rate or extent of mitochondrial electron transport, NADH to ubiquinone. Also known as: regulation of oxidative phosphorylation, NADH to ubiquinone, regulation of complex I (NADH to ubiquinone) References: PMID:23530063 Sources: GOC:TermGenie, GOC:dph, GO_REF:0000058